{
  "gene": "UniProtKB:P24468",
  "gene_name": "COUP transcription factor 2",
  "gene_symbol": "NR2F2",
  "term_id": "GO:0030154",
  "term_label": "cell differentiation"
}